chlorinated hydrocarbon catabolic process [GO:0042205] (biological process) Definition: The chemical reactions and pathways resulting in the breakdown of chlorinated hydrocarbons, compounds derived from hydrocarbons by replacing one or more hydrogen atoms with chlorine atoms. Sources: GOC:ai, GOC:krc Also known as: chlorinated hydrocarbon breakdown, chlorinated hydrocarbon catabolism, chlorinated hydrocarbon degradation Relationships: is a type of GO:0042206 Subtypes: tetrachloroethylene catabolic process [GO:0019337], GO:0042188, trichloroethylene catabolic process [GO:0050696]